L-tryptophan transmembrane transporter activity [GO:0015196] (molecular function) Subtypes: high-affinity tryptophan transmembrane transporter activity [GO:0005300], low-affinity tryptophan transmembrane transporter activity [GO:0022893] Also known as: L-tryptophan transporter activity, L-tryptophan permease activity, valine/tyrosine/tryptophan permease activity Definition: Enables the transfer of L-tryptophan from one side of a membrane to the other. Tryptophan is 2-amino-3-(1H-indol-3-yl)propanoic acid. Relationships: is a type of aromatic amino acid transmembrane transporter activity [GO:0015173]; is_a L-amino acid transmembrane transporter activity [GO:0015179]; is part of tryptophan transport [GO:0015827] Sources: GOC:ai, GOC:mtg_transport, ISBN:0815340729